{
  "term_id": "GO:0008360",
  "gene_name": "Cdc42 effector protein 1",
  "gene_symbol": "CDC42EP1",
  "term_label": "regulation of cell shape",
  "gene": "UniProtKB:Q00587"
}